glucan catabolic process [GO:0009251] (biological process) Sources: GOC:go_curators Relationships: is a type of GO:0000272; is a type of GO:0044042 Definition: The chemical reactions and pathways resulting in the breakdown of glucans, polysaccharides consisting only of glucose residues. Also known as: glucan breakdown, glucan catabolism, glucan degradation Subtypes: glycogen catabolic process [GO:0005980], GO:0005983, alpha-glucan catabolic process [GO:0030980], beta-glucan catabolic process [GO:0051275], pullulan catabolic process [GO:0051678], osmoregulated periplasmic glucan catabolic process [GO:1900726], GO:1901027, GO:2000899